{
  "term_label": "3'-UTR-mediated mRNA stabilization",
  "term_id": "GO:0070935",
  "gene": "UniProtKB:Q13117",
  "gene_symbol": "DAZ2",
  "gene_name": "Deleted in azoospermia protein 2"
}